maintenance of protein location in peroxisome [GO:0072664] (biological process) Definition: Any process in which a protein is maintained in a specific location in a peroxisome, and is prevented from moving elsewhere. Sources: GOC:mah Relationships: is a type of maintenance of protein localization in organelle [GO:0072595]; is part of protein localization to peroxisome [GO:0072662]; occurs in peroxisome [GO:0005777]